{
  "term_label": "Unknown biological process",
  "gene": "UniProtKB:Q96EE4",
  "gene_symbol": "CCDC126",
  "gene_name": "Coiled-coil domain-containing protein 126",
  "term_id": "UNKNOWN:0002"
}